oxidative phosphorylation [GO:0006119] (biological process) Definition: The phosphorylation of ADP to ATP that accompanies the oxidation of a metabolite through the operation of the respiratory chain. Oxidation of compounds establishes a proton gradient across the membrane, providing the energy for ATP synthesis. Regulation: regulated by regulation of oxidative phosphorylation [GO:0002082]; negatively regulated by negative regulation of oxidative phosphorylation [GO:0090324]; positively regulated by GO:1903862 Also known as: respiratory-chain phosphorylation Relationships: is a type of aerobic respiration [GO:0009060]; has part proton motive force-driven ATP synthesis [GO:0015986] Sources: ISBN:0198506732, ISBN:0471331309